{
  "gene": "UniProtKB:Q9HAP6",
  "gene_symbol": "LIN7B",
  "term_id": "GO:0048489",
  "gene_name": "Protein lin-7 homolog B",
  "term_label": "synaptic vesicle transport"
}